interleukin-26 receptor activity [GO:0045508] (molecular function) Relationships: is a type of cytokine receptor activity [GO:0004896]; has part GO:0045512 Definition: Combining with interleukin-26 and transmitting the signal from one side of the membrane to the other to initiate a change in cell activity. Sources: GOC:jl, GOC:signaling Also known as: IL-26 receptor activity, IL-26R